{
  "term_label": "NSL complex",
  "gene": "UniProtKB:Q9P2N6",
  "gene_symbol": "KANSL3",
  "gene_name": "KAT8 regulatory NSL complex subunit 3",
  "term_id": "GO:0044545"
}